{
  "term_label": "ATP-dependent chromatin remodeler activity",
  "gene_name": "Chromodomain-helicase-DNA-binding protein 6",
  "term_id": "GO:0140658",
  "gene_symbol": "CHD6",
  "gene": "UniProtKB:Q8TD26"
}